C-C motif chemokine 2 receptor activity [GO:0038149] (molecular function) Also known as: CCL2 receptor activity Definition: Combining with the C-C motif chemokine 2 (CCL2) and transmitting the signal from one side of the membrane to the other to initiate a change in cell activity. Sources: GOC:bf, GOC:signaling Relationships: is a type of C-C chemokine receptor activity [GO:0016493]; is part of chemokine (C-C motif) ligand 2 signaling pathway [GO:0038148]